regulation of trans-synaptic signaling by BDNF, modulating synaptic transmission [GO:0150035] (biological process) Relationships: is a type of modulation of chemical synaptic transmission [GO:0050804]; regulates trans-synaptic signaling by BDNF, modulating synaptic transmission [GO:0099183] Definition: Any process that modulates the frequency, rate or extent of trans-synaptic signaling by BDNF, modulating synaptic transmission. References: PMID:19448629 Sources: GOC:aruk, GOC:bc Note: Note that this term was created for the SynGO project, and will be obsoleted when the SynGO annotations are made in Noctua.